{
  "gene_name": "Carbonic anhydrase 4",
  "term_label": "carbonate dehydratase activity",
  "term_id": "GO:0004089",
  "gene_symbol": "CA4",
  "gene": "UniProtKB:P22748"
}